{
  "gene_name": "Eukaryotic translation initiation factor 2 subunit 3",
  "term_label": "tRNA binding",
  "gene": "UniProtKB:P41091",
  "term_id": "GO:0000049",
  "gene_symbol": "EIF2S3"
}